negative regulation of glucose mediated signaling pathway [GO:1902660] (biological process) Definition: Any process that stops, prevents or reduces the frequency, rate or extent of glucose mediated signaling pathway. References: PMID:24277933 Sources: GOC:TermGenie, GOC:di, GO_REF:0000058 Also known as: down regulation of glucose mediated signaling pathway, down regulation of glucose mediated signalling, down-regulation of glucose mediated signaling pathway, down-regulation of glucose mediated signalling, downregulation of glucose mediated signaling pathway, downregulation of glucose mediated signalling, negative regulation of glucose mediated signalling, inhibition of glucose mediated signaling pathway, inhibition of glucose mediated signalling Relationships: is a type of negative regulation of signal transduction [GO:0009968]; is a type of regulation of glucose mediated signaling pathway [GO:1902659]; negatively regulates GO:0010255 Subtypes: GO:0110034